regulation of translation in response to oxidative stress [GO:0043556] (biological process) Subtypes: negative regulation of translation in response to oxidative stress [GO:0032938] Relationships: is a type of GO:0032055; BFO_0000050 cellular response to oxidative stress [GO:0034599] Sources: GOC:jl Definition: Any process that modulates the frequency, rate or extent of translation as a result of oxidative stress, a state often resulting from exposure to high levels of reactive oxygen species, e.g. superoxide anions, hydrogen peroxide (H2O2), and hydroxyl radicals.